{
  "gene": "UniProtKB:Q9H0T7",
  "gene_name": "Ras-related protein Rab-17",
  "term_label": "GTPase activity",
  "term_id": "GO:0003924",
  "gene_symbol": "RAB17"
}